mitotic sister chromatid arm separation [GO:1990891] (biological process) Regulation: regulated by GO:1905822; negatively regulated by GO:1905823; positively regulated by GO:1905824 References: PMID:21633354 Definition: The cell cycle process in which sister chromatid arms are physically detached from each other during mitosis. Relationships: is a type of mitotic cell cycle process [GO:1903047]; is part of mitotic sister chromatid separation [GO:0051306]